uracil transmembrane transporter activity [GO:0015210] (molecular function) Definition: Enables the transfer of uracil, 2,4-dioxopyrimidine, from one side of a membrane to the other. Relationships: is_a pyrimidine nucleobase transmembrane transporter activity [GO:0005350]; is part of GO:1903791 Sources: GOC:go_curators Subtypes: GO:0015505 Also known as: uracil/uridine permease activity